{
  "gene": "UniProtKB:Q8TC59",
  "gene_symbol": "PIWIL2",
  "gene_name": "Piwi-like protein 2",
  "term_label": "regulatory ncRNA-mediated gene silencing",
  "term_id": "GO:0031047"
}